{
  "gene_symbol": "CDH2",
  "term_label": "adherens junction organization",
  "gene": "UniProtKB:P19022",
  "gene_name": "Cadherin-2",
  "term_id": "GO:0034332"
}